oxidoreductase activity, acting on paired donors, with incorporation or reduction of molecular oxygen, reduced iron-sulfur protein as one donor, and incorporation of one atom of oxygen [GO:0016713] (molecular function) Also known as: oxidoreductase activity, acting on paired donors, with incorporation or reduction of molecular oxygen, reduced iron-sulphur protein as one donor, and incorporation of one atom of oxygen Relationships: is a type of GO:0004497; is a type of oxidoreductase activity, acting on paired donors, with incorporation or reduction of molecular oxygen [GO:0016705] Subtypes: steroid 11-beta-monooxygenase activity [GO:0004507], GO:0008386, camphor 5-monooxygenase activity [GO:0018683], alkane 1-monooxygenase activity [GO:0018685], GO:0018694, choline monooxygenase activity [GO:0019133], butane monooxygenase activity [GO:0036174], 3-ketosteroid 9-alpha-monooxygenase activity [GO:0036200], ecdysteroid 22-hydroxylase activity [GO:0042767], ecdysteroid 2-hydroxylase activity [GO:0042768], spheroidene monooxygenase activity [GO:0043823], cholestanetetraol 26-dehydrogenase activity [GO:0047748], corticosterone 18-monooxygenase activity [GO:0047783], GO:0052662, GO:0080133, 4-hydroxy-3-all-trans-polyprenylbenzoate oxygenase activity [GO:0106364], 2-methoxy-6-polyprenolphenol 4-hydroxylase activity [GO:0120538] Sources: EC:1.14.15.- Definition: Catalysis of an oxidation-reduction (redox) reaction in which hydrogen or electrons are transferred from reduced iron-sulfur protein and one other donor, and one atom of oxygen is incorporated into one donor.